{
  "term_label": "regulation of transcription by RNA polymerase II",
  "gene_symbol": "ZNF653",
  "gene_name": "Zinc finger protein 653",
  "term_id": "GO:0006357",
  "gene": "UniProtKB:Q96CK0"
}